{
  "term_label": "long-chain fatty acid transmembrane transporter activity",
  "gene_name": "ATP-binding cassette sub-family D member 2",
  "term_id": "GO:0005324",
  "gene_symbol": "ABCD2",
  "gene": "UniProtKB:Q9UBJ2"
}